{
  "gene_symbol": "AGER",
  "gene_name": "Advanced glycosylation end product-specific receptor",
  "term_id": "GO:0031175",
  "term_label": "neuron projection development",
  "gene": "UniProtKB:Q15109"
}